{
  "gene_symbol": "OR8J1",
  "gene": "UniProtKB:Q8NGP2",
  "term_label": "Unknown molecular function",
  "term_id": "UNKNOWN:0001",
  "gene_name": "Olfactory receptor 8J1"
}